{
  "gene_symbol": "GUCY1A2",
  "term_id": "GO:0070482",
  "gene_name": "Guanylate cyclase soluble subunit alpha-2",
  "gene": "UniProtKB:P33402",
  "term_label": "response to oxygen levels"
}